{
  "gene_symbol": "TAX1BP3",
  "term_id": "UNKNOWN:0001",
  "gene_name": "Tax1-binding protein 3",
  "gene": "UniProtKB:O14907",
  "term_label": "Unknown molecular function"
}